{
  "gene_name": "Leucine-rich repeat-containing protein 57",
  "term_label": "Unknown cellular component",
  "term_id": "UNKNOWN:0003",
  "gene_symbol": "LRRC57",
  "gene": "UniProtKB:Q8N9N7"
}